{
  "gene_name": "Interferon-induced transmembrane protein 3",
  "term_label": "negative regulation of viral genome replication",
  "term_id": "GO:0045071",
  "gene": "UniProtKB:Q01628",
  "gene_symbol": "IFITM3"
}